{
  "gene": "UniProtKB:Q8N2K0",
  "term_id": "GO:0047372",
  "term_label": "monoacylglycerol lipase activity",
  "gene_symbol": "ABHD12",
  "gene_name": "Lysophosphatidylserine lipase ABHD12"
}